negative regulation of lysosomal membrane permeability [GO:0097215] (biological process) Definition: Any process that decreases the frequency, rate or extent of the passage or uptake of molecules by the lysosomal membrane. References: PMID:20544854 Sources: GOC:yaf Also known as: negative regulation of lysosome membrane permeability Relationships: is a type of regulation of lysosomal membrane permeability [GO:0097213]; is a type of GO:1905709